{
  "gene": "UniProtKB:Q04864",
  "gene_name": "Proto-oncogene c-Rel",
  "term_id": "GO:0006954",
  "gene_symbol": "REL",
  "term_label": "inflammatory response"
}